{
  "gene": "UniProtKB:Q9HBT7",
  "gene_symbol": "ZNF287",
  "term_id": "GO:0000981",
  "term_label": "DNA-binding transcription factor activity, RNA polymerase II-specific",
  "gene_name": "Zinc finger protein 287"
}